GATOR2 complex [GO:0061700] (cellular component) Relationships: is a type of protein-containing complex [GO:0032991]; is part of Seh1-associated complex [GO:0035859] References: PMID:23723238, PMID:25934700 Sources: GOC:krc, GOC:rb Note: The Rag GTPase complex corresponds to Gtr1-Gtr2 GTPase complex ; GO:1990131. Also known as: SEACAT complex Definition: A multiprotein subcomplex of the GATOR complex that regulates TORC1 signaling by interacting with the Rag GTPase. In human, this complex consists of WDR24, WDR59, MIOS, SEH1L, and SEC13. In S. cerevisiae, this complex is referred to as SEACAT and contains the Sea2p, Sea3p, Sea4p, Seh1p, Sec13p proteins.